{
  "gene_symbol": "VWF",
  "term_label": "cell-substrate adhesion",
  "term_id": "GO:0031589",
  "gene_name": "von Willebrand factor",
  "gene": "UniProtKB:P04275"
}